{
  "term_id": "UNKNOWN:0001",
  "gene_name": "PITH domain-containing protein 1",
  "term_label": "Unknown molecular function",
  "gene": "UniProtKB:Q9GZP4",
  "gene_symbol": "PITHD1"
}